{
  "term_label": "ERAD pathway",
  "gene_name": "Ubiquitin-conjugating enzyme E2 G2",
  "gene_symbol": "UBE2G2",
  "term_id": "GO:0036503",
  "gene": "UniProtKB:P60604"
}